{
  "gene": "UniProtKB:O95295",
  "gene_symbol": "SNAPIN",
  "gene_name": "SNARE-associated protein Snapin",
  "term_id": "GO:0048489",
  "term_label": "synaptic vesicle transport"
}